positive regulation of actin nucleation [GO:0051127] (biological process) Subtypes: positive regulation of Arp2/3 complex-mediated actin nucleation [GO:2000601] Sources: GOC:ai Also known as: up regulation of actin nucleation, up-regulation of actin nucleation, upregulation of actin nucleation, activation of actin nucleation, stimulation of actin nucleation Definition: Any process that activates or increases the frequency, rate or extent of actin nucleation, the initial step in the formation of an actin filament in which actin monomers combine to form a new filament. Relationships: is a type of regulation of actin nucleation [GO:0051125]; is a type of positive regulation of cytoskeleton organization [GO:0051495]; is a type of GO:1902905; positively regulates actin nucleation [GO:0045010]